NK T cell proliferation [GO:0001866] (biological process) Note: Note that NK T cells are a distinct lineage of T cells expressing natural killer cell markers and having T cell receptors characterized by the usage of a restricted repertoire of variable region gene segments. Definition: The expansion of a NK T cell population by cell division. Regulation: regulated by regulation of NK T cell proliferation [GO:0051140]; negatively regulated by negative regulation of NK T cell proliferation [GO:0051141]; positively regulated by positive regulation of NK T cell proliferation [GO:0051142] Also known as: NK T lymphocyte proliferation, NK T-cell proliferation, NK T-lymphocyte proliferation, NKT cell proliferation, NT cell proliferation, natural T cell proliferation, natural killer T cell proliferation Subtypes: NK T cell proliferation involved in immune response [GO:0002289] Relationships: is a type of GO:0046633; is a type of GO:0051132 References: PMID:10704459 Sources: GOC:add, ISBN:0781735149